{
  "gene_symbol": "FAM27E3",
  "term_id": "UNKNOWN:0003",
  "gene": "UniProtKB:Q08E93",
  "gene_name": "Protein FAM27E3",
  "term_label": "Unknown cellular component"
}